{
  "gene": "UniProtKB:Q8N1H7",
  "gene_symbol": "SIX6OS1",
  "term_label": "central element",
  "term_id": "GO:0000801",
  "gene_name": "Protein SIX6OS1"
}